{
  "term_label": "ubiquitin-dependent protein catabolic process",
  "gene_symbol": "AMFR",
  "gene": "UniProtKB:Q9UKV5",
  "term_id": "GO:0006511",
  "gene_name": "E3 ubiquitin-protein ligase AMFR"
}